{
  "gene_symbol": "SMIM21",
  "term_label": "Unknown molecular function",
  "gene": "UniProtKB:Q3B7S5",
  "term_id": "UNKNOWN:0001",
  "gene_name": "Small integral membrane protein 21"
}